{
  "gene_name": "Coiled-coil-helix-coiled-coil-helix domain-containing protein 5",
  "gene": "UniProtKB:Q9BSY4",
  "term_id": "GO:0045333",
  "gene_symbol": "CHCHD5",
  "term_label": "cellular respiration"
}